{
  "gene_name": "Zinc finger and BTB domain-containing protein 49",
  "term_label": "regulation of immune system process",
  "gene": "UniProtKB:Q6ZSB9",
  "term_id": "GO:0002682",
  "gene_symbol": "ZBTB49"
}